antral ovarian follicle growth [GO:0001547] (biological process) Definition: Increase in size of antral follicles due to cell proliferation and/or growth of the antral cavity. Sources: https://www.ncbi.nlm.nih.gov/books/NBK279054/ Relationships: is a type of developmental process involved in reproduction [GO:0003006]; is a type of ovulation cycle process [GO:0022602]; is a type of GO:0048589; is part of ovarian follicle development [GO:0001541] Regulation: regulated by GO:2000387; positively regulated by positive regulation of antral ovarian follicle growth [GO:2000388]